{
  "gene_name": "BTB_POZ domain-containing protein KCTD8",
  "gene_symbol": "KCTD8",
  "term_id": "GO:0008277",
  "term_label": "regulation of G protein-coupled receptor signaling pathway",
  "gene": "UniProtKB:Q6ZWB6"
}